{
  "term_id": "GO:0004499",
  "term_label": "N,N-dimethylaniline monooxygenase activity",
  "gene_name": "Putative dimethylaniline monooxygenase [N-oxide-forming] 6",
  "gene": "UniProtKB:O60774",
  "gene_symbol": "FMO6P"
}